{
  "gene_symbol": "ANGPTL8",
  "gene": "UniProtKB:Q6UXH0",
  "term_label": "Unknown molecular function",
  "term_id": "UNKNOWN:0001",
  "gene_name": "Angiopoietin-like protein 8"
}